{
  "gene": "UniProtKB:Q16623",
  "gene_name": "Syntaxin-1A",
  "term_label": "SNARE complex",
  "term_id": "GO:0031201",
  "gene_symbol": "STX1A"
}